{
  "term_label": "mRNA 3'-UTR binding",
  "gene_name": "Deleted in azoospermia protein 4",
  "gene_symbol": "DAZ4",
  "term_id": "GO:0003730",
  "gene": "UniProtKB:Q86SG3"
}